{
  "gene_name": "Serine_threonine-protein kinase RIO3",
  "gene": "UniProtKB:O14730",
  "term_label": "cytosol",
  "gene_symbol": "RIOK3",
  "term_id": "GO:0005829"
}